regulation of bacterial-type flagellum-dependent cell motility by regulation of motor speed [GO:0071945] (biological process) References: PMID:20371342 Sources: GOC:cilia, GOC:jl Relationships: is a type of GO:1902021 Also known as: regulation of flagellar cell motility by regulation of motor speed, regulation of bacterial-type flagellum cell motility by regulation of motor speed, regulation of bacterial-type flagellar cell motility by regulation of motor speed Definition: A process that modulates flagellum-dependent motility in bacteria by modulating the speed or direction of rotation of a rotary flagellar motor, mediated by interactions between the braking protein.